{
  "gene_symbol": "RABGAP1L",
  "gene_name": "Rab GTPase-activating protein 1-like",
  "term_id": "GO:0005096",
  "gene": "UniProtKB:Q5R372",
  "term_label": "GTPase activator activity"
}